{
  "term_id": "GO:0008289",
  "gene_symbol": "BIN3",
  "gene": "UniProtKB:Q9NQY0",
  "gene_name": "Bridging integrator 3",
  "term_label": "lipid binding"
}